cell surface pattern recognition receptor signaling pathway [GO:0002752] (biological process) Definition: The series of molecular signals initiated by a ligand binding to a cell surface pattern recognition receptor (PRR). PRRs bind pathogen-associated molecular pattern (PAMPs), structures conserved among microbial species. References: PMID:15199967 Sources: GOC:add, GOC:ar, ISBN:0781735149 Also known as: cell surface PAMP receptor signaling pathway, cell surface PRR signaling pathway, cell surface pathogen receptor signaling pathway, cell surface pattern recognition receptor signalling pathway Relationships: is a type of innate immune response activating cell surface receptor signaling pathway [GO:0002220]; is a type of pattern recognition receptor signaling pathway [GO:0002221] Subtypes: toll-like receptor 1 signaling pathway [GO:0034130], cell surface toll-like receptor signaling pathway [GO:0140895]